{
  "gene_symbol": "LBP",
  "term_label": "acute-phase response",
  "gene_name": "Lipopolysaccharide-binding protein",
  "gene": "UniProtKB:P18428",
  "term_id": "GO:0006953"
}